{
  "term_label": "extracellular space",
  "term_id": "GO:0005615",
  "gene_symbol": "WFDC11",
  "gene_name": "Protein WFDC11",
  "gene": "UniProtKB:Q8NEX6"
}